sperm head-tail coupling apparatus [GO:0120212] (cellular component) Relationships: is a type of cellular anatomical structure [GO:0110165] Definition: A centrosome-based structure consisting of two cylindrical microtubule-based centrioles and associated components which anchors the flagellum to the sperm head. Also known as: head-tail coupling apparatus, HTCA, implantation fossa, sperm connecting piece, sperm neck References: PMID:24415959, PMID:30032984 Sources: GOC:krc